{
  "gene_name": "26S proteasome non-ATPase regulatory subunit 9",
  "term_id": "GO:0005634",
  "gene_symbol": "PSMD9",
  "gene": "UniProtKB:O00233",
  "term_label": "nucleus"
}